conjugant formation [GO:0000761] (biological process) Relationships: is a type of adhesion between unicellular organisms [GO:0098610]; is part of conjugation with mutual genetic exchange [GO:0000748] Definition: During conjugation without cellular fusion, the process that results in pairing complementary mating types. Localized morphological, cytological, and cytoskeletal changes connect the mating types without cytoplasmic mixing. Sources: GOC:elh